{
  "gene": "UniProtKB:O75771",
  "gene_name": "DNA repair protein RAD51 homolog 4",
  "gene_symbol": "RAD51D",
  "term_label": "four-way junction DNA binding",
  "term_id": "GO:0000400"
}